tube lumen cavitation [GO:0060605] (BP) Sources: GOC:dph Relationships: is a type of tube formation [GO:0035148] Subtypes: GO:0060604, salivary gland cavitation [GO:0060662] Definition: The formation of a lumen by hollowing out a solid rod or cord. Regulation: regulated by regulation of tube lumen cavitation [GO:1903132]; RO_0002212 by negative regulation of tube lumen cavitation [GO:1903133]